{
  "gene": "UniProtKB:Q16775",
  "gene_name": "Hydroxyacylglutathione hydrolase, mitochondrial",
  "term_id": "GO:0005739",
  "gene_symbol": "HAGH",
  "term_label": "mitochondrion"
}